{
  "term_id": "GO:0008083",
  "gene": "UniProtKB:P11487",
  "gene_symbol": "FGF3",
  "term_label": "growth factor activity",
  "gene_name": "Fibroblast growth factor 3"
}